{
  "term_label": "regulation of cytokine production",
  "term_id": "GO:0001817",
  "gene_name": "ICOS ligand",
  "gene": "UniProtKB:O75144",
  "gene_symbol": "ICOSLG"
}